{
  "gene_symbol": "MBD3L1",
  "gene_name": "Methyl-CpG-binding domain protein 3-like 1",
  "gene": "UniProtKB:Q8WWY6",
  "term_id": "GO:0006346",
  "term_label": "DNA methylation-dependent constitutive heterochromatin formation"
}